{
  "gene_name": "THO complex subunit 6 homolog",
  "term_id": "UNKNOWN:0001",
  "gene": "UniProtKB:Q86W42",
  "term_label": "Unknown molecular function",
  "gene_symbol": "THOC6"
}